prostate gland epithelium morphogenesis [GO:0060740] (biological process) Sources: GOC:dph Definition: The process in which the anatomical structures of epithelia of the prostate gland are generated and organized. An epithelium consists of closely packed cells arranged in one or more layers, that covers the outer surfaces of the body or lines any internal cavity or tube. Relationships: is a type of morphogenesis of an epithelium [GO:0002009]; is a type of developmental process involved in reproduction [GO:0003006]; is part of prostate gland morphogenesis [GO:0060512] Subtypes: GO:0060442, prostatic bud formation [GO:0060513], primary prostatic bud elongation [GO:0060516], prostate epithelial cord elongation [GO:0060523], prostate glandular acinus morphogenesis [GO:0060526]